{
  "gene_symbol": "WWC3",
  "gene": "UniProtKB:Q9ULE0",
  "term_label": "molecular adaptor activity",
  "term_id": "GO:0060090",
  "gene_name": "Protein WWC3"
}